{
  "gene_symbol": "SCN11A",
  "term_label": "cardiac muscle cell action potential involved in contraction",
  "gene": "UniProtKB:Q9UI33",
  "gene_name": "Sodium channel protein type 11 subunit alpha",
  "term_id": "GO:0086002"
}